zinc:proton antiporter activity [GO:0140826] (molecular function) Subtypes: zinc efflux antiporter activity [GO:0015341] Note: Some transporters exchange 1 H+ for a Zn2+ while others are electroneutral and exchange 2 H+. Relationships: is a type of GO:0005385; is a type of GO:0051139 Definition: Enables the transfer of zinc from one side of a membrane to the other according to the reaction: H+(out) + Zn2+(in) = H+(in) + Zn2+(out). References: PMID:19366695, PMID:30893306